GTP guanylyltransferase activity [GO:0047351] (molecular function) Also known as: GTP:GTP guanylyltransferase activity, guanosine-triphosphate guanylyltransferase activity Sources: RHEA:18153 Relationships: is a type of GO:0070568 Definition: Catalysis of the reaction: 2 GTP + H+ = P(1),P(4)-bis(5'-guanosyl) tetraphosphate + diphosphate + H+.